{
  "term_id": "GO:0042110",
  "gene_name": "Trem-like transcript 2 protein",
  "term_label": "T cell activation",
  "gene_symbol": "TREML2",
  "gene": "UniProtKB:Q5T2D2"
}